{
  "gene_symbol": "ZNF423",
  "term_id": "GO:0006355",
  "term_label": "regulation of DNA-templated transcription",
  "gene_name": "Zinc finger protein 423",
  "gene": "UniProtKB:Q2M1K9"
}